{
  "gene_symbol": "SOGA1",
  "gene": "UniProtKB:O94964",
  "gene_name": "Protein SOGA1",
  "term_label": "extracellular space",
  "term_id": "GO:0005615"
}